{
  "gene_name": "Platelet-derived growth factor subunit A",
  "gene": "UniProtKB:P04085",
  "term_id": "GO:0005161",
  "term_label": "platelet-derived growth factor receptor binding",
  "gene_symbol": "PDGFA"
}